{
  "term_id": "UNKNOWN:0001",
  "term_label": "Unknown molecular function",
  "gene_symbol": "RAD52",
  "gene": "UniProtKB:P43351",
  "gene_name": "DNA repair protein RAD52 homolog"
}